chloroplast photosystem I [GO:0030093] (CC) Relationships: is a type of photosystem I [GO:0009522]; is a type of chloroplast thylakoid membrane protein complex [GO:0098807] Sources: GOC:jid, GOC:mtg_sensu Definition: Photosystem located in the chloroplast that functions as a light-dependent plastocyanin-ferredoxin oxidoreductase, transferring electrons from plastocyanin to ferredoxin. An example of this is found in Arabidopsis thaliana.